{
  "gene": "UniProtKB:Q86SX3",
  "term_id": "UNKNOWN:0003",
  "term_label": "Unknown cellular component",
  "gene_symbol": "TEDC1",
  "gene_name": "Tubulin epsilon and delta complex protein 1"
}